{
  "gene_name": "Probable E3 ubiquitin-protein ligase TRIML2",
  "term_id": "GO:0061630",
  "gene_symbol": "TRIML2",
  "term_label": "ubiquitin protein ligase activity",
  "gene": "UniProtKB:Q8N7C3"
}